{
  "term_id": "GO:0030027",
  "gene": "UniProtKB:Q9BR76",
  "term_label": "lamellipodium",
  "gene_name": "Coronin-1B",
  "gene_symbol": "CORO1B"
}